{
  "term_id": "GO:0030424",
  "gene": "UniProtKB:Q92823",
  "gene_symbol": "NRCAM",
  "gene_name": "Neuronal cell adhesion molecule",
  "term_label": "axon"
}